{
  "gene": "UniProtKB:A6NDY0",
  "term_id": "GO:0000288",
  "term_label": "nuclear-transcribed mRNA catabolic process, deadenylation-dependent decay",
  "gene_symbol": "PABPN1L",
  "gene_name": "Embryonic polyadenylate-binding protein 2"
}